protein-containing complex stabilizing activity [GO:0140777] (molecular function) Subtypes: GO:0140778 Relationships: is a type of molecular_function [GO:0003674] Definition: A molecular function that involves direct binding to one of the subunits of a protein-containing complex, thus preventing an interaction with a factor that would promote dissociation of the complex. References: PMID:34040253